{
  "gene": "UniProtKB:Q07820",
  "term_label": "extrinsic apoptotic signaling pathway in absence of ligand",
  "gene_symbol": "MCL1",
  "term_id": "GO:0097192",
  "gene_name": "Induced myeloid leukemia cell differentiation protein Mcl-1"
}